{
  "term_id": "GO:0009880",
  "gene": "UniProtKB:P47902",
  "term_label": "embryonic pattern specification",
  "gene_symbol": "CDX1",
  "gene_name": "Homeobox protein CDX-1"
}